{
  "gene_name": "Chromatin assembly factor 1 subunit B",
  "term_id": "GO:0006334",
  "gene": "UniProtKB:Q13112",
  "term_label": "nucleosome assembly",
  "gene_symbol": "CHAF1B"
}